{
  "gene_symbol": "RIOK2",
  "term_label": "preribosome, small subunit precursor",
  "gene": "UniProtKB:Q9BVS4",
  "term_id": "GO:0030688",
  "gene_name": "Serine_threonine-protein kinase RIO2"
}